{
  "term_id": "GO:0050911",
  "gene_name": "Olfactory receptor 2H2",
  "term_label": "detection of chemical stimulus involved in sensory perception of smell",
  "gene": "UniProtKB:O95918",
  "gene_symbol": "OR2H2"
}